{
  "gene_name": "C-C motif chemokine 22",
  "term_id": "GO:0030335",
  "gene_symbol": "CCL22",
  "gene": "UniProtKB:O00626",
  "term_label": "positive regulation of cell migration"
}